{
  "gene_symbol": "SFTPB",
  "term_label": "Unknown molecular function",
  "gene": "UniProtKB:P07988",
  "gene_name": "Pulmonary surfactant-associated protein B",
  "term_id": "UNKNOWN:0001"
}